rhabdomere development [GO:0042052] (biological process) Also known as: rhabdomere organization Relationships: is a type of organelle organization [GO:0006996]; is part of compound eye photoreceptor development [GO:0042051] Definition: The assembly and arrangement of a rhabdomere within a cell. The rhabdomere is the organelle on the apical surface of a photoreceptor cell that contains the visual pigments. References: PMID:3076112, PMID:3937883